{
  "gene_name": "CCAAT_enhancer-binding protein gamma",
  "gene_symbol": "CEBPG",
  "term_id": "UNKNOWN:0003",
  "gene": "UniProtKB:P53567",
  "term_label": "Unknown cellular component"
}